{
  "gene": "UniProtKB:P0DPB6",
  "term_id": "GO:0006362",
  "gene_symbol": "POLR1D",
  "term_label": "transcription elongation by RNA polymerase I",
  "gene_name": "DNA-directed RNA polymerases I and III subunit RPAC2"
}